fumarate transport [GO:0015741] (biological process) Definition: The directed movement of fumarate into, out of or within a cell, or between cells, by means of some agent such as a transporter or pore. Relationships: is a type of C4-dicarboxylate transport [GO:0015740] Sources: GOC:krc